positive regulation of pyrimidine nucleobase metabolic process [GO:0045985] (biological process) Definition: Any process that activates or increases the frequency, rate or extent of the chemical reactions and pathways involving pyrimidine nucleobases. Sources: GOC:go_curators Also known as: positive regulation of pyrimidine base metabolic process, positive regulation of pyrimidine base metabolism, up regulation of pyrimidine base metabolic process, up-regulation of pyrimidine base metabolic process, upregulation of pyrimidine base metabolic process, activation of pyrimidine base metabolic process, stimulation of pyrimidine base metabolic process Relationships: is_a GO:0019219; is a type of positive regulation of small molecule metabolic process [GO:0062013]; positively regulates pyrimidine nucleobase metabolic process [GO:0006206]